{
  "gene_symbol": "KIR3DL2",
  "term_id": "GO:0140375",
  "term_label": "immune receptor activity",
  "gene": "UniProtKB:P43630",
  "gene_name": "Killer cell immunoglobulin-like receptor 3DL2"
}